{
  "gene_name": "Ribonuclease inhibitor",
  "gene": "UniProtKB:P13489",
  "gene_symbol": "RNH1",
  "term_label": "nucleoplasm",
  "term_id": "GO:0005654"
}